{
  "gene_symbol": "FBXO25",
  "gene": "UniProtKB:Q8TCJ0",
  "term_id": "GO:0016567",
  "gene_name": "F-box only protein 25",
  "term_label": "protein ubiquitination"
}